regulation of protein localization to medial cortex [GO:0106011] (biological process) Definition: Any process that regulates the localization of a protein to the medial cortex. Sources: GOC:hjd Relationships: is a type of regulation of protein localization to cell division site [GO:1901900]; is a type of regulation of protein localization to cell cortex [GO:1904776]; regulates protein localization to medial cortex [GO:0071574] Subtypes: positive regulation of protein localization to medial cortex [GO:0106012], regulation of protein localization to medial cortical node [GO:0120046], negative regulation of protein localization to medial cortex [GO:0140325]